single-stranded DNA helicase activity [GO:0017116] (molecular function) Also known as: single-stranded DNA-dependent ATP-dependent DNA helicase activity, single-stranded DNA-dependent ATPase activity, ssDNA-dependent ATP-dependent DNA helicase activity, ssDNA-dependent ATPase activity Subtypes: single-stranded 3'-5' DNA helicase activity [GO:1990518] Sources: GOC:jl Relationships: is_a DNA helicase activity [GO:0003678] Definition: Catalysis of the reaction: ATP + H2O = ADP + phosphate, in the presence of single-stranded DNA; drives the unwinding of a DNA helix.